{
  "term_label": "canonical Wnt signaling pathway",
  "term_id": "GO:0060070",
  "gene_name": "Protein Wnt-9b",
  "gene_symbol": "WNT9B",
  "gene": "UniProtKB:O14905"
}